{
  "term_label": "regulation of transcription by RNA polymerase II",
  "gene_name": "Zinc finger protein 443",
  "gene_symbol": "ZNF443",
  "term_id": "GO:0006357",
  "gene": "UniProtKB:Q9Y2A4"
}